{
  "term_label": "sarcolemma",
  "gene_name": "Dystrophin",
  "gene": "UniProtKB:P11532",
  "gene_symbol": "DMD",
  "term_id": "GO:0042383"
}